regulation of systemic arterial blood pressure by physical factors [GO:0003045] (biological process) Relationships: is a type of GO:0003073 Sources: GOC:mtg_cardio Also known as: blood pressure regulation by physical factors Subtypes: regulation of systemic arterial blood pressure by stress relaxation [GO:0003046], regulation of systemic arterial blood pressure by capillary fluid shift [GO:0003049] Definition: The regulation of blood pressure mediated by detection of forces within the circulatory system.